{
  "gene": "UniProtKB:Q9UEY8",
  "term_id": "GO:0005856",
  "gene_symbol": "ADD3",
  "term_label": "cytoskeleton",
  "gene_name": "Gamma-adducin"
}